negative regulation of mediator complex assembly [GO:2001177] (biological process) Relationships: is a type of GO:0031333; is a type of regulation of mediator complex assembly [GO:2001176]; negatively regulates mediator complex assembly [GO:0036034] Definition: Any process that stops, prevents or reduces the frequency, rate or extent of mediator complex assembly. Sources: GOC:obol